{
  "gene_symbol": "FAM90A7",
  "gene_name": "Putative protein FAM90A7",
  "term_label": "Unknown molecular function",
  "term_id": "UNKNOWN:0001",
  "gene": "UniProtKB:A6NKC0"
}